{
  "gene_name": "Tectonic-3",
  "term_label": "Unknown molecular function",
  "term_id": "UNKNOWN:0001",
  "gene": "UniProtKB:Q6NUS6",
  "gene_symbol": "TCTN3"
}